{
  "term_id": "GO:0007596",
  "gene_symbol": "PROC",
  "gene": "UniProtKB:P04070",
  "gene_name": "Vitamin K-dependent protein C",
  "term_label": "blood coagulation"
}